SNAP receptor activity [GO:0005484] (MF) Relationships: is a type of GO:0030674; BFO_0000050 membrane fusion [GO:0061025] Also known as: SNARE, Q-SNARE activity, R-SNARE activity, SNAP-25, t-SNARE activity, v-SNARE activity Definition: Acting as a marker to identify a membrane and interacting selectively with one or more SNAREs on another membrane to mediate membrane fusion. References: PMID:14570579 Sources: GOC:mah